cellular response to L-leucine [GO:0071233] (biological process) Sources: GOC:mah Also known as: cellular response to leucine Relationships: is a type of GO:0043201; is a type of cellular response to amino acid stimulus [GO:0071230]; is a type of cellular response to nitrogen compound [GO:1901699]; is a type of cellular response to oxygen-containing compound [GO:1901701] Definition: Any process that results in a change in state or activity of a cell (in terms of movement, secretion, enzyme production, gene expression, etc.) as a result of a L-leucine stimulus.